jasmonic acid and ethylene-dependent systemic resistance, ethylene mediated signaling pathway [GO:0009871] (biological process) Relationships: is a type of ethylene-activated signaling pathway [GO:0009873]; is part of jasmonic acid and ethylene-dependent systemic resistance [GO:0009861] Sources: GOC:jy Definition: The series of molecular signals mediated by ethylene (ethene) involved in jasmonic acid/ethylene dependent systemic resistance. Also known as: ethene mediated signaling pathway (jasmonic acid/ethene-dependent systemic resistance), ethylene mediated signaling pathway (jasmonic acid/ethylene-dependent systemic resistance), jasmonic acid and ethene-dependent systemic resistance, ethene mediated signaling pathway, jasmonic acid/ethene-dependent systemic resistance, ethene mediated signaling pathway, jasmonic acid/ethene-dependent systemic resistance, ethene mediated signalling pathway, jasmonic acid/ethylene-dependent systemic resistance, ethylene mediated signaling pathway, jasmonic acid/ethylene-dependent systemic resistance, ethylene mediated signalling pathway